{
  "term_id": "GO:0140105",
  "gene": "UniProtKB:Q8N6C8",
  "term_label": "interleukin-10-mediated signaling pathway",
  "gene_symbol": "LILRA3",
  "gene_name": "Leukocyte immunoglobulin-like receptor subfamily A member 3"
}